{
  "term_label": "Unknown biological process",
  "gene_name": "Keratin-associated protein 6-3",
  "gene_symbol": "KRTAP6-3",
  "gene": "UniProtKB:Q3LI67",
  "term_id": "UNKNOWN:0002"
}